{
  "term_label": "sperm flagellum",
  "term_id": "GO:0036126",
  "gene_symbol": "GAS8",
  "gene_name": "Dynein regulatory complex subunit 4",
  "gene": "UniProtKB:O95995"
}